{
  "gene_name": "Cytochrome b-245 chaperone 1",
  "term_label": "Unknown biological process",
  "term_id": "UNKNOWN:0002",
  "gene_symbol": "CYBC1",
  "gene": "UniProtKB:Q9BQA9"
}